{
  "term_label": "insulin-like growth factor II binding",
  "gene": "UniProtKB:P24592",
  "term_id": "GO:0031995",
  "gene_symbol": "IGFBP6",
  "gene_name": "Insulin-like growth factor-binding protein 6"
}